{
  "gene_symbol": "PHIP",
  "term_id": "UNKNOWN:0001",
  "gene": "UniProtKB:Q8WWQ0",
  "gene_name": "PH-interacting protein",
  "term_label": "Unknown molecular function"
}